clathrin-sculpted monoamine transport vesicle membrane [GO:0070083] (cellular component) Sources: GOC:mg2 Also known as: clathrin sculpted monoamine constitutive secretory pathway transport vesicle membrane, clathrin sculpted monoamine transport vesicle membrane Relationships: is a type of transport vesicle membrane [GO:0030658]; is a type of GO:0030665; is part of clathrin-sculpted monoamine transport vesicle [GO:0070081] Definition: The lipid bilayer surrounding a clathrin-sculpted monoamine transport vesicle.